{
  "gene_name": "Homologous-pairing protein 2 homolog",
  "gene": "UniProtKB:Q9P2W1",
  "term_id": "GO:0120231",
  "gene_symbol": "PSMC3IP",
  "term_label": "DNA recombinase auxiliary factor complex"
}